{
  "gene": "UniProtKB:P35520",
  "gene_symbol": "CBS",
  "term_id": "GO:0004122",
  "term_label": "cystathionine beta-synthase activity",
  "gene_name": "Cystathionine beta-synthase"
}